{
  "gene": "UniProtKB:Q96KR4",
  "term_id": "GO:0005737",
  "gene_name": "Leishmanolysin-like peptidase",
  "term_label": "cytoplasm",
  "gene_symbol": "LMLN"
}